negative regulation of glutamate metabolic process [GO:2000212] (BP) Subtypes: GO:1901411, negative regulation of L-proline catabolic process to L-glutamate [GO:2001157], negative regulation of ammonia assimilation cycle [GO:2001249] Sources: GOC:sl Relationships: is a type of negative regulation of amino acid metabolic process [GO:0045763]; is a type of negative regulation of small molecule metabolic process [GO:0062014]; is a type of GO:2000211; negatively regulates glutamate metabolic process [GO:0006536] Also known as: negative regulation of glutamate metabolism, negative regulation of glutamic acid metabolic process, negative regulation of glutamic acid metabolism Definition: Any process that stops, prevents, or reduces the frequency, rate or extent of glutamate metabolic process.